{
  "term_id": "UNKNOWN:0001",
  "term_label": "Unknown molecular function",
  "gene": "UniProtKB:Q9H6N6",
  "gene_symbol": "MYH16",
  "gene_name": "Putative uncharacterized protein MYH16"
}